negative regulation of late endosome to lysosome transport [GO:1902823] (biological process) Definition: Any process that stops, prevents or reduces the frequency, rate or extent of late endosome to lysosome transport. Also known as: down regulation of late endosome to lysosome transport, down-regulation of late endosome to lysosome transport, downregulation of late endosome to lysosome transport, inhibition of late endosome to lysosome transport References: PMID:23949442 Sources: GOC:PARL, GOC:TermGenie, GOC:pad, GO_REF:0000058 Relationships: is_a regulation of late endosome to lysosome transport [GO:1902822]; is a type of negative regulation of vacuolar transport [GO:1903336]; negatively regulates late endosome to lysosome transport [GO:1902774]